{
  "term_id": "GO:0042803",
  "gene": "UniProtKB:Q9C035",
  "term_label": "protein homodimerization activity",
  "gene_name": "Tripartite motif-containing protein 5",
  "gene_symbol": "TRIM5"
}